{
  "term_id": "UNKNOWN:0001",
  "gene_name": "Uncharacterized protein C11orf86",
  "term_label": "Unknown molecular function",
  "gene_symbol": "C11orf86",
  "gene": "UniProtKB:A6NJI1"
}